{
  "term_label": "plasma membrane",
  "gene_symbol": "SOS1",
  "term_id": "GO:0005886",
  "gene": "UniProtKB:Q07889",
  "gene_name": "Son of sevenless homolog 1"
}